{
  "gene_name": "Zinc finger and SCAN domain-containing protein 5C",
  "gene_symbol": "ZSCAN5C",
  "term_label": "DNA-binding transcription factor activity, RNA polymerase II-specific",
  "term_id": "GO:0000981",
  "gene": "UniProtKB:A6NGD5"
}